{
  "gene": "UniProtKB:Q9BYH8",
  "gene_name": "NF-kappa-B inhibitor zeta",
  "term_label": "regulation of gene expression",
  "term_id": "GO:0010468",
  "gene_symbol": "NFKBIZ"
}